beta2-adrenergic receptor activity [GO:0004941] (molecular function) Definition: Combining with epinephrine or norepinephrine to initiate a change in cell activity via activation of a G protein, with pharmacological characteristics of beta2-adrenergic receptors. Sources: GOC:mah, IUPHAR_GPCR:1274 Also known as: beta2 adrenoceptor Relationships: is a type of GO:0004939